{
  "gene": "UniProtKB:Q96G28",
  "gene_name": "Cilia- and flagella-associated protein 36",
  "term_label": "ciliary base",
  "gene_symbol": "CFAP36",
  "term_id": "GO:0097546"
}